{
  "gene": "UniProtKB:Q92908",
  "gene_symbol": "GATA6",
  "term_id": "GO:0000981",
  "gene_name": "Transcription factor GATA-6",
  "term_label": "DNA-binding transcription factor activity, RNA polymerase II-specific"
}